{
  "gene_name": "Ubiquitin-conjugating enzyme E2 A",
  "gene": "UniProtKB:P49459",
  "term_id": "GO:0043161",
  "gene_symbol": "UBE2A",
  "term_label": "proteasome-mediated ubiquitin-dependent protein catabolic process"
}